positive regulation of macromolecule biosynthetic process [GO:0010557] (biological process) Sources: GOC:dph, GOC:tb Definition: Any process that increases the rate, frequency or extent of the chemical reactions and pathways resulting in the formation of a macromolecule, any molecule of high relative molecular mass, the structure of which essentially comprises the multiple repetition of units derived, actually or conceptually, from molecules of low relative molecular mass. Subtypes: GO:0010560, GO:0010628, GO:0045345, positive regulation of MHC class II biosynthetic process [GO:0045348], positive regulation of glycogen biosynthetic process [GO:0045725], positive regulation of integrin biosynthetic process [GO:0045726], GO:0046985, positive regulation of (1->3)-beta-D-glucan biosynthetic process [GO:0060635], positive regulation of capsule polysaccharide biosynthetic process [GO:0062085], positive regulation of hyaluronan biosynthetic process [GO:1900127], positive regulation of cutin biosynthetic process [GO:1901959], positive regulation of RNA biosynthetic process [GO:1902680], positive regulation of DNA biosynthetic process [GO:2000573], positive regulation of cellulose biosynthetic process [GO:2001008] Relationships: is a type of positive regulation of biosynthetic process [GO:0009891]; is a type of regulation of macromolecule biosynthetic process [GO:0010556]; is a type of positive regulation of macromolecule metabolic process [GO:0010604]; positively regulates macromolecule biosynthetic process [GO:0009059]